{
  "term_label": "olfactory receptor activity",
  "term_id": "GO:0004984",
  "gene": "UniProtKB:O95013",
  "gene_symbol": "OR4F21",
  "gene_name": "Olfactory receptor 4F21"
}